{
  "gene_symbol": "TNMD",
  "gene": "UniProtKB:Q9H2S6",
  "gene_name": "Tenomodulin",
  "term_label": "negative regulation of angiogenesis",
  "term_id": "GO:0016525"
}